{
  "gene_symbol": "CLASP2",
  "term_label": "establishment of mitotic spindle localization",
  "term_id": "GO:0040001",
  "gene": "UniProtKB:O75122",
  "gene_name": "CLIP-associating protein 2"
}